{
  "gene_symbol": "C1QTNF9B",
  "term_label": "Unknown molecular function",
  "gene_name": "Complement C1q and tumor necrosis factor-related protein 9B",
  "gene": "UniProtKB:B2RNN3",
  "term_id": "UNKNOWN:0001"
}